{
  "term_id": "GO:1903278",
  "gene": "UniProtKB:P58550",
  "term_label": "positive regulation of sodium ion export across plasma membrane",
  "gene_name": "Putative FXYD domain-containing ion transport regulator 8",
  "gene_symbol": "FXYD6P3"
}